{
  "gene": "UniProtKB:P10912",
  "term_label": "positive regulation of cell population proliferation",
  "gene_symbol": "GHR",
  "term_id": "GO:0008284",
  "gene_name": "Growth hormone receptor"
}